{
  "gene_name": "Ras-related protein Rab-22A",
  "term_label": "early endosome",
  "gene_symbol": "RAB22A",
  "gene": "UniProtKB:Q9UL26",
  "term_id": "GO:0005769"
}